{
  "gene_name": "Zinc finger protein 723",
  "term_id": "UNKNOWN:0003",
  "gene_symbol": "ZNF723",
  "gene": "UniProtKB:P0DPD5",
  "term_label": "Unknown cellular component"
}